pyridine-containing compound biosynthetic process [GO:0072525] (biological process) Definition: The chemical reactions and pathways resulting in the formation of a pyridine-containing compound, i.e. any compound that contains pyridine or a formal derivative thereof. Sources: GOC:mah Subtypes: pyridine nucleotide biosynthetic process [GO:0019363], GO:0019805, vitamin B6 biosynthetic process [GO:0042819], pyridine biosynthetic process [GO:0046220], pyridine nucleoside biosynthetic process [GO:0071589], ilicicolin H biosynthetic process [GO:0140781], aspyridone A biosynthetic process [GO:1901518], aspyridone B biosynthetic process [GO:1901521], nicotinate biosynthetic process [GO:1901849], GO:1905004 Relationships: is a type of biosynthetic process [GO:0009058]; is_a pyridine-containing compound metabolic process [GO:0072524] Also known as: pyridine and derivative biosynthetic process, pyridine-containing compound anabolism, pyridine-containing compound biosynthesis, pyridine-containing compound formation, pyridine-containing compound synthesis